{
  "gene": "UniProtKB:P00742",
  "gene_name": "Coagulation factor X",
  "term_id": "GO:0005615",
  "term_label": "extracellular space",
  "gene_symbol": "F10"
}